{
  "term_id": "UNKNOWN:0003",
  "gene_symbol": "SCX",
  "gene": "UniProtKB:Q7RTU7",
  "gene_name": "Basic helix-loop-helix transcription factor scleraxis",
  "term_label": "Unknown cellular component"
}